{
  "gene_name": "WD repeat-containing protein 72",
  "term_id": "GO:0005737",
  "gene_symbol": "WDR72",
  "term_label": "cytoplasm",
  "gene": "UniProtKB:Q3MJ13"
}